{
  "term_label": "Unknown biological process",
  "gene_name": "Olfactory receptor 14A2",
  "gene": "UniProtKB:Q96R54",
  "gene_symbol": "OR14A2",
  "term_id": "UNKNOWN:0002"
}